{
  "term_id": "GO:0045095",
  "gene_symbol": "KRT80",
  "gene": "UniProtKB:Q6KB66",
  "gene_name": "Keratin, type II cytoskeletal 80",
  "term_label": "keratin filament"
}